N-acyl homoserine lactone synthase activity [GO:0061579] (molecular function) Relationships: is a type of GO:0016410 Also known as: autoinducer-1 synthase Sources: RHEA:10096 Definition: Catalysis of the reaction: a fatty acyl-[ACP] + S-adenosyl-L-methionine = an N-acyl-L-homoserine lactone + S-methyl-5'-thioadenosine + holo-[ACP] + H+.